{
  "term_id": "GO:0005929",
  "gene_symbol": "TRPV3",
  "term_label": "cilium",
  "gene": "UniProtKB:Q8NET8",
  "gene_name": "Transient receptor potential cation channel subfamily V member 3"
}